{
  "term_id": "GO:0032036",
  "term_label": "myosin heavy chain binding",
  "gene_symbol": "MYL9",
  "gene": "UniProtKB:P24844",
  "gene_name": "Myosin regulatory light polypeptide 9"
}